{
  "gene": "UniProtKB:Q1A5X6",
  "term_id": "UNKNOWN:0002",
  "gene_symbol": "IQCJ",
  "term_label": "Unknown biological process",
  "gene_name": "IQ domain-containing protein J"
}